{
  "gene_symbol": "SSX9P",
  "gene_name": "Putative protein SSX9",
  "gene": "UniProtKB:Q7RTT3",
  "term_label": "Unknown molecular function",
  "term_id": "UNKNOWN:0001"
}